P-type divalent copper transporter activity [GO:0043682] (molecular function) Definition: Enables the transfer of a solute or solutes from one side of a membrane to the other according to the reaction: ATP + H2O + Cu2+(in) = ADP + phosphate + Cu2+(out). Relationships: is_a GO:0005375; is a type of P-type ion transporter activity [GO:0015662]; is a type of ATPase-coupled monoatomic cation transmembrane transporter activity [GO:0019829] Sources: RHEA:10376 Also known as: copper exporting ATPase activity, copper transmembrane transporter activity, phosphorylative mechanism, copper-translocating P-type ATPase activity, copper-transporting ATPase activity, copper-exporting ATPase activity, Cu(2+)-exporting ATPase activity, Cu2+-exporting ATPase activity